{
  "term_id": "GO:0019210",
  "gene_name": "Glucokinase regulatory protein",
  "term_label": "kinase inhibitor activity",
  "gene": "UniProtKB:Q14397",
  "gene_symbol": "GCKR"
}